{
  "term_label": "positive regulation of somatostatin secretion",
  "term_id": "GO:0090274",
  "gene": "UniProtKB:P09683",
  "gene_name": "Secretin",
  "gene_symbol": "SCT"
}